{
  "gene": "UniProtKB:P47900",
  "gene_symbol": "P2RY1",
  "gene_name": "P2Y purinoceptor 1",
  "term_label": "A1 adenosine receptor binding",
  "term_id": "GO:0031686"
}